{
  "gene": "UniProtKB:Q9NUP9",
  "gene_symbol": "LIN7C",
  "term_label": "cell-cell junction",
  "term_id": "GO:0005911",
  "gene_name": "Protein lin-7 homolog C"
}